{
  "gene_name": "PAT complex subunit CCDC47",
  "term_id": "UNKNOWN:0002",
  "gene_symbol": "CCDC47",
  "term_label": "Unknown biological process",
  "gene": "UniProtKB:Q96A33"
}